{
  "gene": "UniProtKB:Q7Z4H4",
  "term_id": "GO:0010460",
  "term_label": "positive regulation of heart rate",
  "gene_symbol": "ADM2",
  "gene_name": "Protein ADM2"
}